NLRP6 inflammasome complex assembly [GO:0140739] (biological process) Definition: The aggregation, arrangement and bonding together of a set of components to form a NLRP6 inflammasome complex. Relationships: is_a GO:0140632 References: PMID:30674671, PMID:34678144